{
  "gene_symbol": "TIAM1",
  "gene_name": "Rho guanine nucleotide exchange factor TIAM1",
  "term_id": "GO:0005085",
  "gene": "UniProtKB:Q13009",
  "term_label": "guanyl-nucleotide exchange factor activity"
}